{
  "term_id": "GO:0035725",
  "gene_symbol": "SLC6A2",
  "gene": "UniProtKB:P23975",
  "gene_name": "Sodium-dependent noradrenaline transporter",
  "term_label": "sodium ion transmembrane transport"
}